{
  "gene": "UniProtKB:Q9UKI3",
  "term_label": "immune response",
  "term_id": "GO:0006955",
  "gene_name": "Pre-B lymphocyte protein 3",
  "gene_symbol": "VPREB3"
}